{
  "term_id": "GO:0005549",
  "term_label": "odorant binding",
  "gene_symbol": "OR5H2",
  "gene": "UniProtKB:Q8NGV7",
  "gene_name": "Olfactory receptor 5H2"
}